{
  "gene": "UniProtKB:Q02556",
  "term_label": "RNA polymerase II cis-regulatory region sequence-specific DNA binding",
  "gene_symbol": "IRF8",
  "gene_name": "Interferon regulatory factor 8",
  "term_id": "GO:0000978"
}